eoxin D4 synthase activity [GO:0097262] (molecular function) Relationships: is a type of GO:0016755 Definition: Catalysis of the reaction: eoxin C4 = eoxin D4 + 5-L-glutamyl amino acid. References: PMID:18184802, PMID:18647347 Sources: GOC:mw